{
  "term_label": "Unknown cellular component",
  "gene_name": "Uncharacterized protein FAM241A",
  "gene_symbol": "FAM241A",
  "gene": "UniProtKB:Q8N8J7",
  "term_id": "UNKNOWN:0003"
}